{
  "term_label": "plasma membrane",
  "gene_symbol": "FZD6",
  "gene_name": "Frizzled-6",
  "term_id": "GO:0005886",
  "gene": "UniProtKB:O60353"
}